all-trans-8'-apo-beta-carotenal 15,15'-oxygenase activity [GO:0102162] (molecular function) Sources: EC:1.13.11.75, GOC:pz Definition: Catalysis of the reaction: 8'-apo-beta,psi-caroten-8'-al + O2 = all-trans-retinal + 2,6-dimethylocta-2,4,6-trienedial. Relationships: is_a oxidoreductase activity, acting on single donors with incorporation of molecular oxygen, incorporation of two atoms of oxygen [GO:0016702]